renal sodium ion absorption [GO:0070294] (biological process) Definition: A renal system process in which sodium ions are taken up from the collecting ducts and proximal and distal loops of the nephron. In non-mammalian species, absorption may occur in related structures. Sources: GOC:dph, GOC:mah Also known as: nephron sodium ion absorption, renal sodium ion reabsorption Relationships: is a type of renal sodium ion transport [GO:0003096]; is a type of GO:0070293 Subtypes: renal sodium ion absorption involved in negative regulation of renal sodium excretion [GO:0035817]